{
  "term_id": "UNKNOWN:0003",
  "gene_name": "Coiled-coil domain-containing protein 175",
  "term_label": "Unknown cellular component",
  "gene_symbol": "CCDC175",
  "gene": "UniProtKB:P0C221"
}